{
  "gene": "UniProtKB:Q8IX21",
  "term_label": "positive regulation of double-strand break repair",
  "gene_name": "SMC5-SMC6 complex localization factor protein 2",
  "gene_symbol": "SLF2",
  "term_id": "GO:2000781"
}